{
  "gene_name": "Integrator complex subunit 6",
  "gene": "UniProtKB:Q9UL03",
  "term_label": "integrator complex",
  "term_id": "GO:0032039",
  "gene_symbol": "INTS6"
}